positive regulation of cell growth involved in cardiac muscle cell development [GO:0061051] (biological process) Sources: GOC:dph Relationships: is a type of GO:0010613; is a type of GO:0030307; is a type of positive regulation of striated muscle cell differentiation [GO:0051155]; is a type of positive regulation of cardiac muscle tissue growth [GO:0055023]; is a type of regulation of cell growth involved in cardiac muscle cell development [GO:0061050]; positively regulates cell growth involved in cardiac muscle cell development [GO:0061049] Definition: Any process that increases the rate, frequency, or extent of the growth of a cardiac muscle cell, where growth contributes to the progression of the cell over time from its initial formation to its mature state.